{
  "term_label": "regulation of transcription by RNA polymerase II",
  "gene_symbol": "ZNF768",
  "gene_name": "Zinc finger protein 768",
  "term_id": "GO:0006357",
  "gene": "UniProtKB:Q9H5H4"
}